{
  "term_label": "G protein-coupled serotonin receptor activity",
  "gene_name": "5-hydroxytryptamine receptor 6",
  "gene_symbol": "HTR6",
  "gene": "UniProtKB:P50406",
  "term_id": "GO:0004993"
}